{
  "gene": "UniProtKB:P29350",
  "term_id": "GO:0030154",
  "gene_name": "Tyrosine-protein phosphatase non-receptor type 6",
  "term_label": "cell differentiation",
  "gene_symbol": "PTPN6"
}